ocellus pigmentation [GO:0033060] (biological process) Relationships: is a type of pigmentation [GO:0043473] Definition: The deposition or aggregation of coloring matter in an ocellus, a minute simple eye found in many invertebrates. Sources: GOC:mtg_MIT_16mar07